{
  "gene_name": "Coronin-2B",
  "gene_symbol": "CORO2B",
  "gene": "UniProtKB:Q9UQ03",
  "term_id": "GO:0005886",
  "term_label": "plasma membrane"
}